{
  "gene_symbol": "TTC21A",
  "gene": "UniProtKB:Q8NDW8",
  "term_id": "UNKNOWN:0001",
  "term_label": "Unknown molecular function",
  "gene_name": "Tetratricopeptide repeat protein 21A"
}